optic cup structural organization [GO:0003409] (BP) Also known as: optic cup structural organisation Relationships: is a type of GO:0048532; is part of GO:0002072 Sources: GOC:ascb_2009, GOC:dph, GOC:tb Definition: The process that contributes to creating the structural organization of the optic cup. This process pertains to the physical shaping of the rudimentary structure.